{
  "term_id": "GO:0016836",
  "term_label": "hydro-lyase activity",
  "gene": "UniProtKB:Q96EM0",
  "gene_name": "Trans-3-hydroxy-L-proline dehydratase",
  "gene_symbol": "L3HYPDH"
}